morphogenesis of an epithelial sheet [GO:0002011] (biological process) Definition: The process in which the anatomical structures of an epithelial sheet are generated and organized. An epithelial sheet is a flat surface consisting of closely packed epithelial cells. Sources: GOC:jl Relationships: is a type of morphogenesis of an epithelium [GO:0002009] Subtypes: GO:0003344, neural plate elongation [GO:0014022], neural plate thickening [GO:0021991], closure of optic fissure [GO:0061386], epiboly [GO:0090504]